{
  "gene": "UniProtKB:P18507",
  "gene_name": "Gamma-aminobutyric acid receptor subunit gamma-2",
  "gene_symbol": "GABRG2",
  "term_label": "GABA-A receptor complex",
  "term_id": "GO:1902711"
}